{
  "term_label": "phosphoglycerate dehydrogenase activity",
  "term_id": "GO:0004617",
  "gene_symbol": "PHGDH",
  "gene": "UniProtKB:O43175",
  "gene_name": "D-3-phosphoglycerate dehydrogenase"
}